ABC-type transporter activity [GO:0140359] (molecular function) Also known as: ABC transporter, ABC-type efflux permease activity, ABC-type efflux porter activity, ABC-type transmembrane transporter activity, ABC-type uptake permease activity, ATP binding cassette transporter, ATP-binding cassette (ABC) transporter activity, ATP-binding cassette transporter Subtypes: ABC-type guanine transporter activity [GO:0008558], ABC-type xenobiotic transporter activity [GO:0008559], ABC-type ferric iron transporter activity [GO:0015408], GO:0015410, ABC-type molybdate transporter activity [GO:0015412], ABC-type nickel transporter activity [GO:0015413], GO:0015414, ABC-type phosphonate transporter activity [GO:0015416], ABC-type polyamine transporter activity [GO:0015417], ABC-type quaternary ammonium compound transporting activity [GO:0015418], GO:0015419, GO:0015420, ABC-type oligopeptide transporter activity [GO:0015421], ABC-type amino acid transporter activity [GO:0015424], GO:0015430, ABC-type glutathione S-conjugate transporter activity [GO:0015431], GO:0015432, GO:0015434, ABC-type capsular-polysaccharide transporter activity [GO:0015436], GO:0015438, ABC-type heme transporter activity [GO:0015439], GO:0015440, ABC-type protein transporter activity [GO:0015462], ABC-type fatty-acyl-CoA transporter activity [GO:0015607], ABC-type ferric-enterobactin transporter activity [GO:0015624], ABC-type ferric hydroxamate transporter activity [GO:0015625], ABC-type zinc transporter activity [GO:0015633], ABC-type betaine transporter activity [GO:0031458], ABC-type choline transporter activity [GO:0033266], ABC-type sterol transporter activity [GO:0034041], GO:0042959, ABC-type carbohydrate transporter activity [GO:0043211], GO:0044604, ABC-type thiosulfate transporter activity [GO:0102025], GO:0140394, ABC-type iron-sulfur cluster transporter activity [GO:0140481], ABC-type sodium transporter activity [GO:0140679], GO:0160080, ABC-type tungstate transporter activity [GO:1901238], ABC-type doxorubicin transporter activity [GO:1901242], GO:1905948 Definition: Primary active transporter characterized by two nucleotide-binding domains and two transmembrane domains. Uses the energy generated from ATP hydrolysis to drive the transport of a substance across a membrane. Relationships: is a type of ATPase-coupled transmembrane transporter activity [GO:0042626] References: PMID:26517899